{
  "gene_name": "Long-chain-fatty-acid--CoA ligase 4",
  "gene_symbol": "ACSL4",
  "term_label": "endoplasmic reticulum",
  "gene": "UniProtKB:O60488",
  "term_id": "GO:0005783"
}